beta-zeacarotene catabolic process [GO:1901817] (biological process) Also known as: beta-zeacarotene breakdown, beta-zeacarotene catabolism, beta-zeacarotene degradation References: PMID:3710717 Sources: GOC:TermGenie, GOC:yaf, UniPathway:UPA00805 Relationships: is a type of GO:0016118; is a type of carotene catabolic process [GO:0016121] Definition: The chemical reactions and pathways resulting in the breakdown of beta-zeacarotene.